{
  "gene_symbol": "GOSR1",
  "term_id": "GO:0005797",
  "gene": "UniProtKB:O95249",
  "gene_name": "Golgi SNAP receptor complex member 1",
  "term_label": "Golgi medial cisterna"
}